(+)-lariciresinol biosynthetic process [GO:1902132] (biological process) References: PMID:8910615, PMID:9872995 Sources: GOC:TermGenie Relationships: is a type of GO:0009807; is a type of primary alcohol biosynthetic process [GO:0034309]; is a type of GO:0046189; is a type of ether biosynthetic process [GO:1901503] Definition: The chemical reactions and pathways resulting in the formation of (+)-lariciresinol. Also known as: (+)-lariciresinol anabolism, (+)-lariciresinol biosynthesis, (+)-lariciresinol formation, (+)-lariciresinol synthesis